{
  "gene": "UniProtKB:Q8IWY9",
  "gene_symbol": "CDAN1",
  "term_label": "Unknown molecular function",
  "gene_name": "Codanin-1",
  "term_id": "UNKNOWN:0001"
}